{
  "gene_symbol": "CXorf49B",
  "term_label": "Unknown cellular component",
  "term_id": "UNKNOWN:0003",
  "gene": "UniProtKB:A8MYA2",
  "gene_name": "Uncharacterized protein CXorf49"
}